anterior lateral line ganglion neuron differentiation [GO:0048908] (biological process) Relationships: is a type of GO:0048891; is part of GO:0048907 Definition: The process in which a relatively unspecialized cell acquires specialized features of a neuron of the anterior lateral line ganglion. References: PMID:15018940